central nervous system neuron development [GO:0021954] (BP) Relationships: is a type of neuron development [GO:0048666]; is part of central nervous system neuron differentiation [GO:0021953] Definition: The process whose specific outcome is the progression of a neuron whose cell body is located in the central nervous system, from initial commitment of the cell to a neuronal fate, to the fully functional differentiated neuron. Sources: GOC:cls, GOC:dgh, GOC:dph, GOC:jid, GO_REF:0000021 Subtypes: forebrain neuron development [GO:0021884], GO:0098749